positive regulation of octopamine signaling pathway involved in response to food [GO:2000141] (biological process) Definition: Any process that activates or increases the frequency, rate or extent of octopamine signaling pathway involved in response to food. References: PMID:19609300 Sources: GOC:mah Also known as: positive regulation of octopamine signalling pathway involved in response to food Relationships: is a type of positive regulation of response to food [GO:0032097]; is a type of positive regulation of octopamine signaling pathway [GO:2000130]; is a type of regulation of octopamine signaling pathway involved in response to food [GO:2000139]; positively regulates GO:0071935